fosmidomycin transmembrane transporter activity [GO:0042898] (molecular function) Definition: Enables the transfer of fosmidomycin, a phosphonic acid derivative with potent activity against Gram-negative organisms, from one side of a membrane to the other. Also known as: fosmidomycin transporter activity Relationships: is_a GO:0042887; is part of fosmidomycin transport [GO:0042894] References: PMID:12543685 Sources: GOC:jl